{
  "gene_name": "Tumor necrosis factor receptor superfamily member 19",
  "gene_symbol": "TNFRSF19",
  "term_label": "signaling receptor activity",
  "term_id": "GO:0038023",
  "gene": "UniProtKB:Q9NS68"
}